{
  "gene_name": "Solute carrier family 35 member G5",
  "gene": "UniProtKB:Q96KT7",
  "term_id": "GO:0016020",
  "term_label": "membrane",
  "gene_symbol": "SLC35G5"
}